{
  "gene_symbol": "C15orf62",
  "gene_name": "Uncharacterized protein C15orf62, mitochondrial",
  "gene": "UniProtKB:A8K5M9",
  "term_label": "small GTPase binding",
  "term_id": "GO:0031267"
}